{
  "gene": "UniProtKB:Q15722",
  "term_id": "GO:0005886",
  "gene_name": "Leukotriene B4 receptor 1",
  "term_label": "plasma membrane",
  "gene_symbol": "LTB4R"
}